tensidol B biosynthetic process [GO:1900608] (biological process) Sources: GOC:TermGenie, GOC:di Regulation: regulated by GO:1900710; RO_0002212 by GO:1900711; RO_0002213 by positive regulation of tensidol B biosynthetic process [GO:1900712] Also known as: tensidol B anabolism, tensidol B biosynthesis, tensidol B formation, tensidol B synthesis Definition: The chemical reactions and pathways resulting in the formation of tensidol B. Relationships: is a type of ketone biosynthetic process [GO:0042181]; is_a amide biosynthetic process [GO:0043604]; is a type of secondary metabolite biosynthetic process [GO:0044550]; is a type of carboxylic acid biosynthetic process [GO:0046394]